{
  "gene_symbol": "KYAT3",
  "gene": "UniProtKB:Q6YP21",
  "gene_name": "Kynurenine--oxoglutarate transaminase 3",
  "term_label": "mitochondrion",
  "term_id": "GO:0005739"
}